{
  "gene": "UniProtKB:Q8TDL5",
  "gene_name": "BPI fold-containing family B member 1",
  "term_id": "UNKNOWN:0003",
  "term_label": "Unknown cellular component",
  "gene_symbol": "BPIFB1"
}